{
  "term_id": "UNKNOWN:0002",
  "gene_symbol": "AADACL2",
  "gene_name": "Arylacetamide deacetylase-like 2",
  "term_label": "Unknown biological process",
  "gene": "UniProtKB:Q6P093"
}